P1 peroxisome [GO:0019819] (cellular component) Also known as: peroxisome vesicle Relationships: is a type of GO:0005777 Note: Note that this peroxisome assembly pathway is described in the yeast Yarrowia lipolytica. See also the cellular component terms 'P2 peroxisome ; GO:0019820', 'P3 peroxisome ; GO:0019821', 'P4 peroxisome ; GO:0019822', 'P5 peroxisome ; GO:0019823', and 'P6 peroxisome ; GO:0019824'. References: PMID:10629216 Definition: A subform of peroxisome that corresponds to an intermediate in a peroxisome assembly pathway, which operates by conversion of peroxisomal subforms in the direction P1, P2 -> P3 -> P4 -> P5 -> P6. P1 peroxisomes are distinguished from the other subforms on the bases of buoyant density and protein content; they contain fewer peroxisomal proteins than the other subforms.